{
  "term_id": "GO:0004722",
  "gene_name": "Dual specificity protein phosphatase CDC14B",
  "gene_symbol": "CDC14B",
  "gene": "UniProtKB:O60729",
  "term_label": "protein serine/threonine phosphatase activity"
}